RCAF complex [GO:0035059] (cellular component) Definition: A protein complex that facilitates the assembly of nucleosomes on to newly synthesized DNA. In Drosophila, the complex comprises ASF1 and histones H3 and H4. Also known as: replication-coupling assembly factor complex References: PMID:10591219 Sources: GOC:bf Relationships: is a type of GO:0140513